{
  "term_id": "GO:0051560",
  "gene_symbol": "ANXA6",
  "term_label": "mitochondrial calcium ion homeostasis",
  "gene_name": "Annexin A6",
  "gene": "UniProtKB:P08133"
}